alpha9-beta1 integrin-tenascin complex [GO:0071082] (cellular component) Relationships: is a type of plasma membrane protein complex [GO:0098797] References: PMID:9565552 Also known as: ITGA9-ITGB1-TNC complex Definition: A protein complex that consists of an alpha9-beta1 integrin complex bound to the extracellular matrix protein tenascin.